cyanuric acid amidohydrolase activity [GO:0018753] (molecular function) Definition: Catalysis of the reaction: cyanurate + H2O = 1-carboxybiuret + H+. Sources: EC:3.5.2.15 Relationships: is a type of hydrolase activity, acting on carbon-nitrogen (but not peptide) bonds, in cyclic amides [GO:0016812]